{
  "term_label": "extracellular space",
  "term_id": "GO:0005615",
  "gene_name": "Lithostathine-1-alpha",
  "gene_symbol": "REG1A",
  "gene": "UniProtKB:P05451"
}